{
  "gene_name": "Putative uncharacterized protein encoded by LINC00308",
  "term_id": "UNKNOWN:0003",
  "gene": "UniProtKB:Q8TCZ7",
  "gene_symbol": "LINC00308",
  "term_label": "Unknown cellular component"
}